{
  "term_id": "GO:0004556",
  "gene_symbol": "AMY2A",
  "term_label": "alpha-amylase activity",
  "gene": "UniProtKB:P04746",
  "gene_name": "Pancreatic alpha-amylase"
}